ocellus morphogenesis [GO:0048816] (biological process) Relationships: is a type of post-embryonic animal morphogenesis [GO:0009886]; is a type of GO:0090596; is part of eye-antennal disc morphogenesis [GO:0007455]; is part of ocellus development [GO:0008056] Sources: http://fly.ebi.ac.uk/.bin/cvreport2?id=FBcv0004540 Definition: The process in which the anatomical structures of the ocellus are generated and organized. The ocellus is a simple visual organ of insects.